{
  "term_label": "nucleus",
  "gene_name": "Piwi-like protein 3",
  "term_id": "GO:0005634",
  "gene": "UniProtKB:Q7Z3Z3",
  "gene_symbol": "PIWIL3"
}